regulation of antibacterial peptide biosynthetic process [GO:0002808] (BP) Definition: Any process that modulates the frequency, rate, or extent of antibacterial peptide biosynthesis. Relationships: is a type of regulation of antibacterial peptide production [GO:0002786]; is a type of regulation of antimicrobial peptide biosynthetic process [GO:0002805]; regulates GO:0002780 Subtypes: negative regulation of antibacterial peptide biosynthetic process [GO:0002809], regulation of biosynthetic process of antibacterial peptides active against Gram-negative bacteria [GO:0002813], regulation of biosynthetic process of antibacterial peptides active against Gram-positive bacteria [GO:0002816], GO:0006963 Sources: GOC:add